mannosyl-inositol phosphorylceramide metabolic process [GO:0006675] (biological process) Relationships: is a type of inositol phosphoceramide metabolic process [GO:0006673]; is a type of glycosphingolipid metabolic process [GO:0006687] Subtypes: mannosyl-inositol phosphorylceramide biosynthetic process [GO:0051999] Also known as: MIPC metabolic process, MIPC metabolism, mannose inositol phosphoceramide metabolic process, mannose inositol phosphoceramide metabolism, mannose-inositol-P-ceramide (MIPC) metabolic process, mannose-inositol-P-ceramide (MIPC) metabolism, mannosyl-inositol-phosphorylceramide metabolism Definition: The chemical reactions and pathways involving mannosyl-inositol phosphorylceramide, any lipid with a phosphodiester bridge between an inositol residue and the ceramide group which contains a phosphoryl (-P(O)=) groups and a mannose derivative. Sources: GOC:ai